{
  "term_id": "GO:0090110",
  "gene": "UniProtKB:O94855",
  "gene_name": "Protein transport protein Sec24D",
  "term_label": "COPII-coated vesicle cargo loading",
  "gene_symbol": "SEC24D"
}